{
  "gene_name": "Solute carrier family 41 member 3",
  "term_id": "UNKNOWN:0002",
  "term_label": "Unknown biological process",
  "gene_symbol": "SLC41A3",
  "gene": "UniProtKB:Q96GZ6"
}